{
  "term_id": "UNKNOWN:0001",
  "term_label": "Unknown molecular function",
  "gene": "UniProtKB:Q96QU8",
  "gene_symbol": "XPO6",
  "gene_name": "Exportin-6"
}